{
  "gene_symbol": "WIPI1",
  "gene": "UniProtKB:Q5MNZ9",
  "term_label": "phagophore assembly site membrane",
  "term_id": "GO:0034045",
  "gene_name": "WD repeat domain phosphoinositide-interacting protein 1"
}